{
  "gene": "UniProtKB:P23743",
  "gene_name": "Diacylglycerol kinase alpha",
  "term_label": "diacylglycerol metabolic process",
  "gene_symbol": "DGKA",
  "term_id": "GO:0046339"
}